{
  "gene_symbol": "KIAA0232",
  "term_label": "Unknown cellular component",
  "gene_name": "Uncharacterized protein KIAA0232",
  "term_id": "UNKNOWN:0003",
  "gene": "UniProtKB:Q92628"
}